{
  "gene_symbol": "H2BC5",
  "term_label": "nucleus",
  "term_id": "GO:0005634",
  "gene": "UniProtKB:P58876",
  "gene_name": "Histone H2B type 1-D"
}